{
  "term_id": "GO:0030667",
  "gene_name": "Islet cell autoantigen 1",
  "term_label": "secretory granule membrane",
  "gene_symbol": "ICA1",
  "gene": "UniProtKB:Q05084"
}